{
  "gene_symbol": "NXPE3",
  "gene": "UniProtKB:Q969Y0",
  "gene_name": "NXPE family member 3",
  "term_id": "UNKNOWN:0002",
  "term_label": "Unknown biological process"
}